calcium ion-regulated exocytosis of neurotransmitter [GO:0048791] (biological process) Subtypes: fast, calcium ion-dependent exocytosis of neurotransmitter [GO:0098746], slow, calcium ion-dependent exocytosis of neurotransmitter [GO:0098747], presynaptic dense core vesicle exocytosis [GO:0099525] Definition: The release of a neurotransmitter into the synaptic cleft by exocytosis of synaptic vesicles, where the release step is dependent on a rise in cytosolic calcium ion levels. Relationships: is a type of synaptic vesicle exocytosis [GO:0016079]; is a type of GO:0017156 Sources: GOC:curators Regulation: regulated by GO:1903233; RO_0002212 by GO:1903234; positively regulated by positive regulation of calcium ion-dependent exocytosis of neurotransmitter [GO:1903235]